dGTPase activity [GO:0008832] (molecular function) Definition: Catalysis of the reaction: dGTP + H2O = 2'-deoxyguanosine + 2 H+ + triphosphate. Sources: RHEA:15193 Also known as: deoxyguanosinetriphosphate triphosphohydrolase activity, dGTP triphosphohydrolase activity, deoxy-GTPase activity, deoxyguanosine 5-triphosphate triphosphohydrolase activity, deoxyguanosine triphosphatase activity, deoxyguanosine triphosphate triphosphohydrolase activity Relationships: is a type of GO:0016793